negative regulation of positive chemotaxis to cAMP by DIF-2 [GO:0061129] (biological process) Definition: Any process that decreases the rate, frequency, or extent of directed movement of a motile cell or organism up a concentration gradient of 3',5'-cAMP by the action of DIF-2. DIF-2 is a chlorinated alkylphenone. Sources: GOC:dph Relationships: is a type of regulation of positive chemotaxis to cAMP by DIF-2 [GO:0061121]; is a type of negative regulation of positive chemotaxis to cAMP by chlorinated alkylphenone [GO:0061125]